{
  "gene_symbol": "SEC61A2",
  "gene": "UniProtKB:Q9H9S3",
  "gene_name": "Protein transport protein Sec61 subunit alpha isoform 2",
  "term_id": "GO:0005784",
  "term_label": "Sec61 translocon complex"
}